{
  "gene_name": "Translocating chain-associated membrane protein 1",
  "term_id": "UNKNOWN:0001",
  "term_label": "Unknown molecular function",
  "gene": "UniProtKB:Q15629",
  "gene_symbol": "TRAM1"
}